{
  "gene_name": "Mitogen-activated protein kinase 10",
  "gene": "UniProtKB:P53779",
  "term_label": "JUN kinase activity",
  "term_id": "GO:0004705",
  "gene_symbol": "MAPK10"
}